spectrosome [GO:0045170] (cellular component) Sources: GOC:bf Definition: A germline specific spherical organelle, rich in membrane skeletal proteins. Precursor to the fusome. Relationships: is a type of intracellular membraneless organelle [GO:0043232]; is part of cytoplasm [GO:0005737]